threonine transport [GO:0015826] (biological process) Relationships: is a type of neutral amino acid transport [GO:0015804]; is a type of GO:0046942; is a type of nitrogen compound transport [GO:0071705] Also known as: L-threonine transport Definition: The directed movement of threonine, (2R*,3S*)-2-amino-3-hydroxybutanoic acid, into, out of or within a cell, or between cells, by means of some agent such as a transporter or pore. Subtypes: L-threonine import across plasma membrane [GO:1903807] Sources: GOC:ai